{
  "term_id": "GO:0030490",
  "gene_symbol": "SRFBP1",
  "gene_name": "Serum response factor-binding protein 1",
  "term_label": "maturation of SSU-rRNA",
  "gene": "UniProtKB:Q8NEF9"
}